{
  "gene": "UniProtKB:Q15532",
  "gene_symbol": "SS18",
  "term_label": "positive regulation of transcription by RNA polymerase II",
  "gene_name": "Protein SSXT",
  "term_id": "GO:0045944"
}